{
  "term_id": "UNKNOWN:0001",
  "gene_symbol": "TRAJ61",
  "gene_name": "T cell receptor alpha joining 61 (non-functional) (Fragment)",
  "gene": "UniProtKB:A0A075B708",
  "term_label": "Unknown molecular function"
}